{
  "term_id": "GO:0005634",
  "gene_name": "Protein mono-ADP-ribosyltransferase PARP12",
  "term_label": "nucleus",
  "gene": "UniProtKB:Q9H0J9",
  "gene_symbol": "PARP12"
}